{
  "gene": "UniProtKB:Q08AD1",
  "gene_name": "Calmodulin-regulated spectrin-associated protein 2",
  "gene_symbol": "CAMSAP2",
  "term_id": "GO:0036449",
  "term_label": "microtubule minus-end"
}